{
  "term_id": "GO:0033106",
  "gene_name": "Trafficking protein particle complex subunit 3-like protein",
  "gene_symbol": "TRAPPC3L",
  "term_label": "cis-Golgi network membrane",
  "gene": "UniProtKB:Q5T215"
}